{
  "gene_name": "ADP-ribosylation factor-like protein 2",
  "gene_symbol": "ARL2",
  "gene": "UniProtKB:P36404",
  "term_id": "GO:0005737",
  "term_label": "cytoplasm"
}